{
  "gene_name": "Metallothionein-1X",
  "term_id": "GO:0071280",
  "term_label": "cellular response to copper ion",
  "gene_symbol": "MT1X",
  "gene": "UniProtKB:P80297"
}